{
  "gene": "UniProtKB:Q6P5Q4",
  "term_id": "GO:0007015",
  "gene_name": "Leiomodin-2",
  "gene_symbol": "LMOD2",
  "term_label": "actin filament organization"
}